{
  "term_id": "GO:0033065",
  "gene_name": "DNA repair protein RAD51 homolog 3",
  "gene_symbol": "RAD51C",
  "term_label": "Rad51C-XRCC3 complex",
  "gene": "UniProtKB:O43502"
}